{
  "gene_symbol": "RNF7",
  "term_id": "GO:0005634",
  "term_label": "nucleus",
  "gene": "UniProtKB:Q9UBF6",
  "gene_name": "RING-box protein 2"
}